{
  "gene_name": "Mitochondrial import inner membrane translocase subunit TIM44",
  "term_label": "protein-folding chaperone binding",
  "term_id": "GO:0051087",
  "gene": "UniProtKB:O43615",
  "gene_symbol": "TIMM44"
}